membrane bending [GO:0097753] (biological process) Also known as: membrane curvature Definition: A membrane organization process resulting in the bending of a membrane. Relationships: is a type of membrane organization [GO:0061024] Subtypes: clathrin-mediated membrane bending [GO:0097754] Sources: GOC:krc, GOC:pr, GOC:vw, Wikipedia:Membrane_curvature